{
  "gene_symbol": "NTN1",
  "term_label": "RNA polymerase II cis-regulatory region sequence-specific DNA binding",
  "gene": "UniProtKB:O95631",
  "term_id": "GO:0000978",
  "gene_name": "Netrin-1"
}